negative regulation of antibody-dependent cellular cytotoxicity [GO:0001814] (BP) Relationships: is_a negative regulation of type IIa hypersensitivity [GO:0001797]; is a type of regulation of antibody-dependent cellular cytotoxicity [GO:0001813]; is a type of negative regulation of leukocyte mediated cytotoxicity [GO:0001911]; negatively regulates antibody-dependent cellular cytotoxicity [GO:0001788] Definition: Any process that stops, prevents, or reduces the rate of antibody-dependent cellular cytotoxicity. Sources: GOC:add, ISBN:0781735149 Also known as: down regulation of antibody-dependent cellular cytotoxicity, down-regulation of antibody-dependent cellular cytotoxicity, downregulation of antibody-dependent cellular cytotoxicity, negative regulation of antibody dependent cell death, negative regulation of antibody dependent cell killing, negative regulation of antibody-dependent cell death, negative regulation of antibody-dependent cell killing, inhibition of antibody-dependent cellular cytotoxicity